{
  "gene": "UniProtKB:Q9BZB8",
  "term_label": "cytoplasm",
  "gene_symbol": "CPEB1",
  "term_id": "GO:0005737",
  "gene_name": "Cytoplasmic polyadenylation element-binding protein 1"
}